{
  "gene_symbol": "ZBTB7A",
  "term_id": "GO:0000978",
  "gene": "UniProtKB:O95365",
  "term_label": "RNA polymerase II cis-regulatory region sequence-specific DNA binding",
  "gene_name": "Zinc finger and BTB domain-containing protein 7A"
}